{
  "gene_name": "Mothers against decapentaplegic homolog 1",
  "term_label": "anatomical structure morphogenesis",
  "gene_symbol": "SMAD1",
  "term_id": "GO:0009653",
  "gene": "UniProtKB:Q15797"
}